{
  "gene_symbol": "CCNC",
  "gene_name": "Cyclin-C",
  "term_id": "GO:0005634",
  "gene": "UniProtKB:P24863",
  "term_label": "nucleus"
}